{
  "term_id": "GO:0071014",
  "term_label": "post-mRNA release spliceosomal complex",
  "gene_name": "Probable splicing factor YJU2B",
  "gene": "UniProtKB:P13994",
  "gene_symbol": "YJU2B"
}